{
  "gene": "UniProtKB:P55198",
  "gene_symbol": "MLLT6",
  "gene_name": "Protein AF-17",
  "term_label": "nucleus",
  "term_id": "GO:0005634"
}